{
  "term_id": "GO:0032809",
  "gene": "UniProtKB:Q03721",
  "term_label": "neuronal cell body membrane",
  "gene_name": "Potassium voltage-gated channel subfamily C member 4",
  "gene_symbol": "KCNC4"
}